sour taste receptor activity [GO:0033040] (molecular function) Definition: Combining with soluble sour compounds to initiate a change in cell activity. These receptors are responsible for the sense of sour taste. Sources: GOC:mah Relationships: is a type of taste receptor activity [GO:0008527]; is part of detection of chemical stimulus involved in sensory perception of sour taste [GO:0001581]